{
  "gene_name": "Zinc finger protein PLAGL2",
  "term_label": "sequence-specific DNA binding",
  "gene_symbol": "PLAGL2",
  "term_id": "GO:0043565",
  "gene": "UniProtKB:Q9UPG8"
}